{
  "term_id": "GO:0006325",
  "gene_symbol": "UBN1",
  "term_label": "chromatin organization",
  "gene_name": "Ubinuclein-1",
  "gene": "UniProtKB:Q9NPG3"
}